{
  "term_id": "UNKNOWN:0002",
  "gene_name": "Putative transporter SVOPL",
  "gene_symbol": "SVOPL",
  "term_label": "Unknown biological process",
  "gene": "UniProtKB:Q8N434"
}